{
  "gene_name": "Olfactory receptor 2A5",
  "gene": "UniProtKB:Q96R48",
  "term_label": "plasma membrane",
  "gene_symbol": "OR2A5",
  "term_id": "GO:0005886"
}